{
  "gene_symbol": "OTUD6A",
  "term_label": "cysteine-type deubiquitinase activity",
  "term_id": "GO:0004843",
  "gene_name": "OTU domain-containing protein 6A",
  "gene": "UniProtKB:Q7L8S5"
}